{
  "term_id": "GO:0004930",
  "gene_symbol": "LPAR3",
  "gene_name": "Lysophosphatidic acid receptor 3",
  "gene": "UniProtKB:Q9UBY5",
  "term_label": "G protein-coupled receptor activity"
}